{
  "term_label": "Unknown molecular function",
  "gene_symbol": "CCDC28A-AS1",
  "term_id": "UNKNOWN:0001",
  "gene": "UniProtKB:A0A096LPI5",
  "gene_name": "Putative uncharacterized protein CCDC28A-AS1"
}